{
  "gene_symbol": "SEMA4A",
  "gene_name": "Semaphorin-4A",
  "term_label": "plasma membrane",
  "gene": "UniProtKB:Q9H3S1",
  "term_id": "GO:0005886"
}